{
  "term_label": "cell migration",
  "term_id": "GO:0016477",
  "gene_symbol": "CDH24",
  "gene_name": "Cadherin-24",
  "gene": "UniProtKB:Q86UP0"
}